{
  "term_label": "protein kinase activator activity",
  "gene_name": "Serine_threonine-protein kinase STK11",
  "term_id": "GO:0030295",
  "gene": "UniProtKB:Q15831",
  "gene_symbol": "STK11"
}